{
  "gene_symbol": "IMPA1",
  "term_id": "GO:0007165",
  "term_label": "signal transduction",
  "gene_name": "Inositol monophosphatase 1",
  "gene": "UniProtKB:P29218"
}